phospholipase inhibitor activity [GO:0004859] (molecular function) Sources: GOC:ai, GOC:rl Subtypes: phospholipase A2 inhibitor activity [GO:0019834], phospholipase D inhibitor activity [GO:0060961], phospholipase C inhibitor activity [GO:0160186] Relationships: is a type of GO:0055102; negatively regulates phospholipase activity [GO:0004620] Definition: Binds to and stops, prevents or reduces the activity of a phospholipase, an enzyme that catalyzes of the hydrolysis of a phospholipid.